{
  "term_id": "GO:0000786",
  "term_label": "nucleosome",
  "gene": "UniProtKB:P68431",
  "gene_symbol": "H3C12",
  "gene_name": "Histone H3.1"
}